{
  "gene": "UniProtKB:P13591",
  "gene_name": "Neural cell adhesion molecule 1",
  "term_label": "neuron projection",
  "gene_symbol": "NCAM1",
  "term_id": "GO:0043005"
}